{
  "gene_symbol": "ARHGEF40",
  "term_id": "GO:0007411",
  "gene_name": "Rho guanine nucleotide exchange factor 40",
  "term_label": "axon guidance",
  "gene": "UniProtKB:Q8TER5"
}